{
  "gene": "UniProtKB:Q9H2B4",
  "gene_symbol": "SLC26A1",
  "term_label": "oxalate transmembrane transporter activity",
  "gene_name": "Sulfate anion transporter 1",
  "term_id": "GO:0019531"
}